{
  "gene_symbol": "PRPS1",
  "term_label": "5-phosphoribose 1-diphosphate biosynthetic process",
  "term_id": "GO:0006015",
  "gene": "UniProtKB:P60891",
  "gene_name": "Ribose-phosphate pyrophosphokinase 1"
}